{
  "gene_symbol": "HDAC3",
  "term_label": "histone deacetylase activity",
  "term_id": "GO:0004407",
  "gene_name": "Histone deacetylase 3",
  "gene": "UniProtKB:O15379"
}